negative regulation of microtubule nucleation [GO:1905833] (BP) Relationships: is a type of GO:0010968; is a type of negative regulation of microtubule polymerization [GO:0031115]; RO_0002212 GO:0007020 Also known as: down regulation of microtubule nucleation, down-regulation of microtubule nucleation, downregulation of microtubule nucleation, inhibition of microtubule nucleation Definition: Any process that stops, prevents or reduces the frequency, rate or extent of microtubule nucleation. References: PMID:27689799 Sources: GOC:TermGenie, GO_REF:0000058